abequosyltransferase activity [GO:0047600] (molecular function) Relationships: is a type of hexosyltransferase activity [GO:0016758] Sources: EC:2.4.1.60, MetaCyc:ABEQUOSYLTRANSFERASE-RXN Also known as: CDP-abequose:D-mannosyl-L-rhamnosyl-D-galactose-1-diphospholipid D-abequosyltransferase activity, trihexose diphospholipid abequosyltransferase activity Definition: Catalysis of the reaction: CDP-abequose + D-mannosyl-L-rhamnosyl-D-galactose-1-diphospholipid = CDP + D-abequosyl-D-mannosyl-rhamnosyl-D-galactose-1-diphospholipid.